{
  "gene_symbol": "LRRC4C",
  "term_label": "postsynaptic density membrane",
  "gene": "UniProtKB:Q9HCJ2",
  "gene_name": "Leucine-rich repeat-containing protein 4C",
  "term_id": "GO:0098839"
}